{
  "gene": "UniProtKB:O95256",
  "gene_symbol": "IL18RAP",
  "gene_name": "Interleukin-18 receptor accessory protein",
  "term_label": "plasma membrane",
  "term_id": "GO:0005886"
}